{
  "gene_symbol": "AIDA",
  "term_id": "GO:0016020",
  "gene_name": "Axin interactor, dorsalization-associated protein",
  "term_label": "membrane",
  "gene": "UniProtKB:Q96BJ3"
}